{
  "term_label": "Unknown cellular component",
  "gene_name": "Ig-like domain-containing protein (Fragment)",
  "gene_symbol": "LOC102724971",
  "term_id": "UNKNOWN:0003",
  "gene": "UniProtKB:A0A087WW49"
}